{
  "term_label": "cytosol",
  "gene_name": "Ethylmalonyl-CoA decarboxylase",
  "gene": "UniProtKB:Q9NTX5",
  "term_id": "GO:0005829",
  "gene_symbol": "ECHDC1"
}